{
  "gene": "UniProtKB:Q96J66",
  "gene_name": "ATP-binding cassette sub-family C member 11",
  "term_label": "transmembrane transport",
  "gene_symbol": "ABCC11",
  "term_id": "GO:0055085"
}